{
  "gene": "UniProtKB:Q8WYA0",
  "gene_symbol": "IFT81",
  "gene_name": "Intraflagellar transport protein 81 homolog",
  "term_id": "GO:0042073",
  "term_label": "intraciliary transport"
}